{
  "gene_symbol": "NTF4",
  "gene_name": "Neurotrophin-4",
  "term_id": "GO:0007169",
  "gene": "UniProtKB:P34130",
  "term_label": "cell surface receptor protein tyrosine kinase signaling pathway"
}